{
  "term_id": "GO:0005634",
  "gene": "UniProtKB:Q14872",
  "term_label": "nucleus",
  "gene_name": "Metal regulatory transcription factor 1",
  "gene_symbol": "MTF1"
}